{
  "term_label": "Unknown biological process",
  "gene_symbol": "VPS9D1",
  "term_id": "UNKNOWN:0002",
  "gene_name": "VPS9 domain-containing protein 1",
  "gene": "UniProtKB:Q9Y2B5"
}